{
  "term_label": "olfactory receptor activity",
  "gene_symbol": "OR2B11",
  "gene": "UniProtKB:Q5JQS5",
  "term_id": "GO:0004984",
  "gene_name": "Olfactory receptor 2B11"
}